{
  "term_label": "antigen binding",
  "term_id": "GO:0003823",
  "gene": "UniProtKB:P0CF74",
  "gene_name": "Immunoglobulin lambda constant 6",
  "gene_symbol": "IGLC6"
}